{
  "term_id": "GO:0035869",
  "term_label": "ciliary transition zone",
  "gene": "UniProtKB:Q9P0N5",
  "gene_symbol": "TMEM216",
  "gene_name": "Transmembrane protein 216"
}